{
  "term_label": "Unknown molecular function",
  "term_id": "UNKNOWN:0001",
  "gene_name": "Multivesicular body subunit 12A",
  "gene_symbol": "MVB12A",
  "gene": "UniProtKB:Q96EY5"
}